{
  "term_label": "GTPase activity",
  "term_id": "GO:0003924",
  "gene_name": "Ras-related protein Rab-33B",
  "gene": "UniProtKB:Q9H082",
  "gene_symbol": "RAB33B"
}